maintenance of centrosome location [GO:0051661] (biological process) Definition: Any process in which a centrosome is maintained in a specific location within a cell and prevented from moving elsewhere. Relationships: is a type of centrosome localization [GO:0051642]; is a type of maintenance of organelle location [GO:0051657] Also known as: maintenance of centrosome localization Sources: GOC:ai, GOC:dph, GOC:tb